extracellular vesicle biogenesis [GO:0140112] (biological process) Definition: The assembly and secretion a set of components to form an extracellular vesicule, a membrane-bounded vesicle that is released into the extracellular region. Extracellular vesicles include exosomes, microvesicles and apoptotic bodies, based on the mechanism by which they are released from cells and differentiated based on their size and content. References: PMID:28736435 Also known as: extracellular vesicle assembly Relationships: is a type of cellular component biogenesis [GO:0044085] Subtypes: extracellular exosome biogenesis [GO:0097734], extracellular microvesicle biogenesis [GO:0140113]